{
  "term_label": "regulation of transcription by RNA polymerase II",
  "gene_symbol": "EGR3",
  "gene_name": "Early growth response protein 3",
  "gene": "UniProtKB:Q06889",
  "term_id": "GO:0006357"
}